{
  "gene_symbol": "ADCY4",
  "term_label": "plasma membrane",
  "gene": "UniProtKB:Q8NFM4",
  "gene_name": "Adenylate cyclase type 4",
  "term_id": "GO:0005886"
}